{
  "term_label": "Unknown biological process",
  "term_id": "UNKNOWN:0002",
  "gene": "UniProtKB:Q86YJ5",
  "gene_name": "E3 ubiquitin-protein ligase MARCHF9",
  "gene_symbol": "MARCHF9"
}